{
  "gene_name": "Alpha-hemoglobin-stabilizing protein",
  "term_id": "GO:0006457",
  "gene": "UniProtKB:Q9NZD4",
  "gene_symbol": "AHSP",
  "term_label": "protein folding"
}